Tor2-Mei2-Ste11 complex [GO:0034064] (cellular component) References: PMID:17046992 Sources: GOC:vw Definition: A protein complex that contains the transcription factor Ste11 and the RNA binding protein Mei2; involved in regulation of conjugation in fission yeast. Relationships: is a type of GO:0140513